{
  "gene": "UniProtKB:Q92599",
  "term_id": "GO:0005940",
  "gene_name": "Septin-8",
  "term_label": "septin ring",
  "gene_symbol": "SEPTIN8"
}